cellular response to corticosteroid stimulus [GO:0071384] (biological process) Definition: Any process that results in a change in state or activity of a cell (in terms of movement, secretion, enzyme production, gene expression, etc.) as a result of a corticosteroid hormone stimulus. A corticosteroid is a steroid hormone that is produced in the adrenal cortex. Corticosteroids are involved in a wide range of physiologic systems such as stress response, immune response and regulation of inflammation, carbohydrate metabolism, protein catabolism, blood electrolyte levels, and behavior. They include glucocorticoids and mineralocorticoids. Relationships: is a type of GO:0031960; is a type of GO:0071383 Sources: GOC:mah Subtypes: cellular response to glucocorticoid stimulus [GO:0071385], GO:0071389